{
  "gene": "UniProtKB:Q6J272",
  "term_label": "Unknown biological process",
  "gene_symbol": "FAM166A",
  "gene_name": "Protein FAM166A",
  "term_id": "UNKNOWN:0002"
}